{
  "gene": "UniProtKB:Q99717",
  "term_id": "GO:0030154",
  "gene_name": "Mothers against decapentaplegic homolog 5",
  "term_label": "cell differentiation",
  "gene_symbol": "SMAD5"
}